{
  "term_label": "heparin binding",
  "gene": "UniProtKB:P29279",
  "term_id": "GO:0008201",
  "gene_name": "CCN family member 2",
  "gene_symbol": "CCN2"
}